{
  "term_id": "GO:0001525",
  "gene": "UniProtKB:Q15389",
  "term_label": "angiogenesis",
  "gene_name": "Angiopoietin-1",
  "gene_symbol": "ANGPT1"
}